symbiont-mediated perturbation of host innate immune response [GO:0052167] (biological process) Definition: A process in which a symbiont alters or subverts the innate immune response of the host organism; the innate immune response is the host's first line of defense against infection. The host is defined as the larger of the organisms involved in a symbiotic interaction. Sources: GOC:mtg_pamgo_17jul06 Subtypes: symbiont-mediated perturbation of host natural killer cell mediated immune response [GO:0039671], symbiont-mediated suppression of host dendritic cell mediated immune response [GO:0039673], symbiont-mediated perturbation of host inflammatory response [GO:0052032], GO:0052088, symbiont-mediated perturbation of host resistance gene-dependent defense response [GO:0052158], symbiont defense to host-produced reactive oxygen species [GO:0052164], GO:0052170, GO:0140404 Relationships: is a type of symbiont-mediated perturbation of host immune response [GO:0052553] Also known as: modulation by organism of innate immune response in other organism involved in symbiotic interaction, modulation by symbiont of host innate immunity, modulation of host innate immune response, perturbation of host innate immune response